{
  "gene_symbol": "RYK",
  "gene_name": "Tyrosine-protein kinase RYK",
  "term_id": "GO:0007409",
  "gene": "UniProtKB:P34925",
  "term_label": "axonogenesis"
}